{
  "gene": "UniProtKB:Q99447",
  "gene_symbol": "PCYT2",
  "gene_name": "Ethanolamine-phosphate cytidylyltransferase",
  "term_label": "ethanolamine-phosphate cytidylyltransferase activity",
  "term_id": "GO:0004306"
}